{
  "gene_symbol": "VTI1A",
  "term_label": "intra-Golgi vesicle-mediated transport",
  "gene": "UniProtKB:Q96AJ9",
  "term_id": "GO:0006891",
  "gene_name": "Vesicle transport through interaction with t-SNAREs homolog 1A"
}